{
  "term_label": "phosphatidylcholine-sterol O-acyltransferase activator activity",
  "gene_name": "Apolipoprotein A-IV",
  "term_id": "GO:0060228",
  "gene_symbol": "APOA4",
  "gene": "UniProtKB:P06727"
}